{
  "gene": "UniProtKB:Q8WVZ7",
  "gene_symbol": "RNF133",
  "term_id": "GO:0005789",
  "term_label": "endoplasmic reticulum membrane",
  "gene_name": "E3 ubiquitin-protein ligase RNF133"
}